{
  "gene_symbol": "CCDC134",
  "term_label": "endoplasmic reticulum lumen",
  "gene": "UniProtKB:Q9H6E4",
  "term_id": "GO:0005788",
  "gene_name": "Coiled-coil domain-containing protein 134"
}